{
  "gene_name": "Killer cell immunoglobulin-like receptor 3DS1",
  "gene_symbol": "KIR3DS1",
  "term_id": "GO:0140375",
  "term_label": "immune receptor activity",
  "gene": "UniProtKB:Q14943"
}